cyclin K-CDK13 complex [GO:0002945] (cellular component) Also known as: CycK/Cdk13 complex Definition: A protein complex consisting of cyclin Kand cyclin-dependent kinase 13 (CDK13). Cyclins are characterized by periodicity in protein abundance throughout the cell cycle. Cyclin-dependent kinases represent a family of serine/threonine protein kinases that become active upon binding to a cyclin regulatory partner. References: PMID:22012619 Relationships: is a type of cyclin-dependent protein kinase holoenzyme complex [GO:0000307]